interleukin-12 receptor complex [GO:0042022] (cellular component) Definition: A protein complex that binds interleukin-12 and that consists of, at a minimum, a dimeric interleukin and its two receptor subunits as well as optional additional kinase subunits. References: PMID:10971505 Sources: GOC:ebc, GOC:mah Also known as: IL-12 receptor complex, IL12RB1-IL12RB2 complex Relationships: is a type of plasma membrane signaling receptor complex [GO:0098802]